{
  "gene": "UniProtKB:Q6NSW7",
  "term_label": "nucleus",
  "term_id": "GO:0005634",
  "gene_symbol": "NANOGP8",
  "gene_name": "Homeobox protein NANOGP8"
}